{
  "gene_name": "Major facilitator superfamily domain-containing protein 8",
  "term_label": "iodide transmembrane transporter activity",
  "gene_symbol": "MFSD8",
  "term_id": "GO:0015111",
  "gene": "UniProtKB:Q8NHS3"
}